{
  "gene": "UniProtKB:Q99720",
  "gene_symbol": "SIGMAR1",
  "term_id": "UNKNOWN:0002",
  "term_label": "Unknown biological process",
  "gene_name": "Sigma non-opioid intracellular receptor 1"
}